regulation of metaphase/anaphase transition of meiosis II [GO:1905189] (biological process) Also known as: regulation of meiosis II metaphase/anaphase transition Definition: Any process that modulates the frequency, rate or extent of metaphase/anaphase transition of meiosis II. References: PMID:21389117 Sources: GOC:TermGenie, GO_REF:0000058 Subtypes: GO:1905190, positive regulation of metaphase/anaphase transition of meiosis II [GO:1905191] Relationships: is a type of regulation of metaphase/anaphase transition of meiotic cell cycle [GO:1902102]; regulates metaphase/anaphase transition of meiosis II [GO:1990950]